regulation of translation at postsynapse [GO:0140245] (biological process) Relationships: is a type of regulation of translation at synapse [GO:0140243]; BFO_0000066 postsynapse [GO:0098794] References: PMID:20427644 Note: Note that this term was created for the SynGO project, and will be obsoleted when the SynGO annotations are made in Noctua. Subtypes: GO:0099578 Definition: Any process that regulates translation occurring at the postsynapse.